{
  "gene": "UniProtKB:Q96NL1",
  "gene_name": "Transmembrane protein 74",
  "gene_symbol": "TMEM74",
  "term_label": "Unknown molecular function",
  "term_id": "UNKNOWN:0001"
}